{
  "gene": "UniProtKB:Q86YW7",
  "term_label": "extracellular space",
  "term_id": "GO:0005615",
  "gene_symbol": "GPHB5",
  "gene_name": "Glycoprotein hormone beta-5"
}